{
  "gene_name": "SAFB-like transcription modulator",
  "gene": "UniProtKB:Q9NWH9",
  "term_id": "GO:0005634",
  "gene_symbol": "SLTM",
  "term_label": "nucleus"
}